{
  "gene": "UniProtKB:Q12829",
  "gene_name": "Ras-related protein Rab-40B",
  "gene_symbol": "RAB40B",
  "term_id": "GO:0005886",
  "term_label": "plasma membrane"
}